{
  "term_label": "extracellular space",
  "gene": "UniProtKB:Q9NZH8",
  "term_id": "GO:0005615",
  "gene_symbol": "IL36G",
  "gene_name": "Interleukin-36 gamma"
}